{
  "gene_name": "Pikachurin",
  "gene": "UniProtKB:Q63HQ2",
  "term_label": "synapse",
  "term_id": "GO:0045202",
  "gene_symbol": "EGFLAM"
}